{
  "gene_name": "Ubiquitin-conjugating enzyme E2 U",
  "term_id": "GO:0061631",
  "gene": "UniProtKB:Q5VVX9",
  "term_label": "ubiquitin conjugating enzyme activity",
  "gene_symbol": "UBE2U"
}